{
  "term_label": "protein processing",
  "gene": "UniProtKB:Q96BI3",
  "gene_name": "Gamma-secretase subunit APH-1A",
  "gene_symbol": "APH1A",
  "term_id": "GO:0016485"
}